immunoglobulin transcytosis in epithelial cells [GO:0002414] (biological process) Subtypes: GO:0002415, IgG immunoglobulin transcytosis in epithelial cells mediated by FcRn immunoglobulin receptor [GO:0002416] Definition: The process of transporting immunoglobulin, via transcytosis, from one side of an epithelial cell to the other. Relationships: is a type of GO:0045056 References: PMID:16048543 Sources: GOC:add, ISBN:0781735149, ISBN:081533642X